IgM B cell receptor complex [GO:0071755] (cellular component) Also known as: membrane-bound IgM, surface IgM Note: Note that an IgM immunoglobulin complex has the function of antigen binding if a suitable antigen is available. Relationships: is a type of GO:0019815; is a type of GO:0071753 References: PMID:20176268 Sources: GOC:add, ISBN:0781765196 Definition: An IgM immunoglobulin complex that is present in the plasma membrane of B cells and is composed of two identical immunoglobulin heavy chains of the IgM isotype and two identical immunoglobulin light chains and a signaling subunit, a heterodimer of the Ig-alpha and Ig-beta proteins.